{
  "gene_symbol": "CAV1",
  "term_label": "focal adhesion",
  "term_id": "GO:0005925",
  "gene_name": "Caveolin-1",
  "gene": "UniProtKB:Q03135"
}